{
  "term_id": "GO:0016324",
  "gene_symbol": "UMOD",
  "term_label": "apical plasma membrane",
  "gene_name": "Uromodulin",
  "gene": "UniProtKB:P07911"
}